{
  "gene_symbol": "RPH3A",
  "term_label": "postsynaptic membrane",
  "gene_name": "Rabphilin-3A",
  "gene": "UniProtKB:Q9Y2J0",
  "term_id": "GO:0045211"
}